protein O-linked glycosylation via xylose [GO:0180064] (biological process) Also known as: protein O-linked xylosylation Relationships: is a type of GO:0006493 References: PMID:22117070 Definition: A glycoprotein biosynthetic process starting with the covalent linkage of a xylose via a beta-glycosidic bond to the oxygen atom of a serine or a threonine side chain in a protein, which can be further elongated with the sequential addition of sugar units resulting in the formation of a protein O-linked glycan. Subtypes: GO:0015012, heparin proteoglycan biosynthetic process [GO:0030210], chondroitin sulfate proteoglycan biosynthetic process [GO:0050650], dermatan sulfate proteoglycan biosynthetic process [GO:0050651], GO:0120532